carpel morphogenesis [GO:0048445] (biological process) Sources: GOC:go_curators Definition: The process in which the anatomical structures of the carpel are generated and organized. Relationships: is a type of floral organ morphogenesis [GO:0048444]; is part of carpel development [GO:0048440]